{
  "term_label": "ammonium transmembrane transport",
  "gene_name": "Ammonium transporter Rh type B",
  "term_id": "GO:0072488",
  "gene": "UniProtKB:Q9H310",
  "gene_symbol": "RHBG"
}